positive regulation of RNA binding [GO:1905216] (biological process) Definition: Any process that activates or increases the frequency, rate or extent of RNA binding. References: PMID:25116364 Sources: GOC:PARL, GOC:TermGenie, GOC:bf, GO_REF:0000059 Also known as: up regulation of RNA binding, up-regulation of RNA binding, upregulation of RNA binding, activation of RNA binding Relationships: is a type of positive regulation of binding [GO:0051099]; positively regulates RNA binding [GO:0003723] Subtypes: positive regulation of mRNA binding [GO:1902416]